{
  "gene_name": "LHFPL tetraspan subfamily member 5 protein",
  "term_label": "detection of mechanical stimulus involved in sensory perception",
  "gene": "UniProtKB:Q8TAF8",
  "term_id": "GO:0050974",
  "gene_symbol": "LHFPL5"
}